{
  "term_id": "GO:0004876",
  "term_label": "complement component C3a receptor activity",
  "gene": "UniProtKB:Q16581",
  "gene_symbol": "C3AR1",
  "gene_name": "C3a anaphylatoxin chemotactic receptor"
}